{
  "gene": "UniProtKB:Q6ZPB5",
  "gene_symbol": "SDIM1",
  "term_id": "UNKNOWN:0001",
  "gene_name": "Stress-responsive DNAJB4-interacting membrane protein 1",
  "term_label": "Unknown molecular function"
}